{
  "term_label": "Unknown biological process",
  "gene": "UniProtKB:Q8IXR5",
  "gene_name": "Protein FAM178B",
  "gene_symbol": "FAM178B",
  "term_id": "UNKNOWN:0002"
}